{
  "gene": "UniProtKB:Q6PUV4",
  "term_label": "SNARE complex",
  "gene_name": "Complexin-2",
  "term_id": "GO:0031201",
  "gene_symbol": "CPLX2"
}